{
  "gene": "UniProtKB:P43320",
  "gene_symbol": "CRYBB2",
  "term_id": "GO:0005212",
  "gene_name": "Beta-crystallin B2",
  "term_label": "structural constituent of eye lens"
}